inositol-4,5-bisphosphate 5-phosphatase activity [GO:0030487] (molecular function) Definition: Catalysis of the reaction: 1D-myo-inositol 4,5-bisphosphate + H2O = 1D-myo-inositol 4-phosphate + phosphate. Sources: GOC:mah Relationships: is a type of inositol bisphosphate phosphatase activity [GO:0016312]